{
  "gene": "UniProtKB:Q6P9H4",
  "term_label": "protein-macromolecule adaptor activity",
  "gene_name": "Connector enhancer of kinase suppressor of ras 3",
  "term_id": "GO:0030674",
  "gene_symbol": "CNKSR3"
}